{
  "term_label": "Unknown molecular function",
  "gene_name": "WD repeat-containing protein 11",
  "term_id": "UNKNOWN:0001",
  "gene_symbol": "WDR11",
  "gene": "UniProtKB:Q9BZH6"
}